{
  "gene_name": "Interleukin-1 receptor-associated kinase 3",
  "gene_symbol": "IRAK3",
  "gene": "UniProtKB:Q9Y616",
  "term_label": "plasma membrane",
  "term_id": "GO:0005886"
}